cytoplasmic actin-based contraction involved in forward cell motility [GO:0060328] (biological process) Definition: The actin filament-based movement by which cytoplasmic actin filaments slide past one another resulting in a contraction that propels the cell in the direction that has been defined as the front of the cell. Sources: GOC:dph Also known as: cytoplasmic actin-based contraction involved in forward cell locomotion Relationships: is a type of cytoplasmic actin-based contraction involved in cell motility [GO:0060327]